{
  "gene_symbol": "PNLIP",
  "gene": "UniProtKB:P16233",
  "term_id": "GO:0034375",
  "gene_name": "Pancreatic triacylglycerol lipase",
  "term_label": "high-density lipoprotein particle remodeling"
}